{
  "gene_name": "Putative uncharacterized protein FLJ42213",
  "term_label": "Unknown molecular function",
  "gene_symbol": "Q6ZVQ6",
  "gene": "UniProtKB:Q6ZVQ6",
  "term_id": "UNKNOWN:0001"
}